{
  "term_label": "Unknown molecular function",
  "gene": "UniProtKB:O96007",
  "gene_symbol": "MOCS2",
  "term_id": "UNKNOWN:0001",
  "gene_name": "Molybdopterin synthase catalytic subunit"
}